{
  "gene_symbol": "IL17RD",
  "term_label": "Unknown cellular component",
  "term_id": "UNKNOWN:0003",
  "gene_name": "Interleukin-17 receptor D",
  "gene": "UniProtKB:Q8NFM7"
}